{
  "gene": "UniProtKB:P37837",
  "term_label": "nucleus",
  "gene_symbol": "TALDO1",
  "gene_name": "Transaldolase",
  "term_id": "GO:0005634"
}